{
  "gene_name": "Protein phosphatase 1E",
  "term_id": "GO:0051496",
  "gene_symbol": "PPM1E",
  "term_label": "positive regulation of stress fiber assembly",
  "gene": "UniProtKB:Q8WY54"
}